{
  "gene_symbol": "ELOVL6",
  "gene_name": "Elongation of very long chain fatty acids protein 6",
  "term_id": "GO:0030148",
  "gene": "UniProtKB:Q9H5J4",
  "term_label": "sphingolipid biosynthetic process"
}